N-succinyltransferase activity [GO:0016749] (molecular function) Subtypes: 5-aminolevulinate synthase activity [GO:0003870], 2,3,4,5-tetrahydropyridine-2,6-dicarboxylate N-succinyltransferase activity [GO:0008666], arginine N-succinyltransferase activity [GO:0008791] Relationships: is a type of GO:0016410; is a type of GO:0016748 Sources: GOC:ai Definition: Catalysis of the transfer of a succinyl group to a nitrogen atom on the acceptor molecule.